{
  "term_label": "Unknown biological process",
  "gene_name": "T cell receptor alpha joining 4 (Fragment)",
  "gene": "UniProtKB:A0A075B6Z5",
  "gene_symbol": "TRAJ4",
  "term_id": "UNKNOWN:0002"
}